{
  "term_id": "GO:0007189",
  "gene_name": "G-protein coupled receptor 12",
  "gene": "UniProtKB:P47775",
  "gene_symbol": "GPR12",
  "term_label": "adenylate cyclase-activating G protein-coupled receptor signaling pathway"
}